{
  "gene_name": "Ubiquitin-like modifier-activating enzyme 6",
  "gene": "UniProtKB:A0AVT1",
  "gene_symbol": "UBA6",
  "term_id": "GO:0006511",
  "term_label": "ubiquitin-dependent protein catabolic process"
}